vanillate monooxygenase activity [GO:0018489] (molecular function) Definition: Catalysis of the reaction: H+ + NADH + O2 + vanillate = 3,4-dihydroxybenzoate + formaldehyde + H2O + NAD+. Sources: EC:1.14.13.82, RHEA:13021 Note: Note that this was EC:1.2.3.12. Also known as: vanillate demethylase (aerobic) activity, vanillate demethylase activity, 4-hydroxy-3-methoxybenzoate demethylase activity, vanillate:oxygen oxidoreductase (demethylating) Relationships: is a type of oxidoreductase activity, acting on paired donors, with incorporation or reduction of molecular oxygen, NAD(P)H as one donor, and incorporation of one atom of oxygen [GO:0016709]; is a type of demethylase activity [GO:0032451]